floral meristem growth [GO:0010451] (biological process) Regulation: regulated by regulation of floral meristem growth [GO:0010080] Definition: The increase in size or mass of a floral meristem, a population of undifferentiated cells in a plant that gives rise to a flower. Relationships: is a type of developmental process involved in reproduction [GO:0003006]; is a type of meristem growth [GO:0035266]; is part of flower development [GO:0009908] Sources: GOC:tb